symbiont-mediated perturbation of host defenses [GO:0030682] (biological process) Sources: GOC:mtg_pamgo_17jul06 Subtypes: GO:0044414, symbiont-mediated perturbation of host phagocytosis [GO:0052067], symbiont-mediated perturbation of host resistance gene-dependent defense response [GO:0052158] Definition: A process in which a symbiont alters or subverts the normal execution of a host organism's defense response. The host defense response is mounted by the host in response to the presence of the symbiont. The host is defined as the larger of the organisms involved in a symbiotic interaction. Also known as: evasion or tolerance of defense response of other organism involved in symbiotic interaction, mitigation of host defenses by symbiont, perturbation of host defenses by symbiont, avoidance of defenses of other organism involved in symbiotic interaction, avoidance of host defences, avoidance of host defenses, evasion of host defence response, evasion of other organism defence response, evasion or tolerance of host defense response, avoidance of defenses of other organism during symbiotic interaction, evasion or tolerance of defense response of other organism during symbiotic interaction, evasion or tolerance of defenses of other organism, evasion or tolerance of defenses of other organism during symbiotic interaction, evasion or tolerance of defenses of other organism involved in symbiotic interaction, evasion or tolerance of host defenses Relationships: is a type of symbiont-mediated response to host defenses [GO:0052200]